epithelial cell morphogenesis involved in gastrulation [GO:0003381] (biological process) Relationships: is a type of epithelial cell morphogenesis [GO:0003382]; is part of gastrulation [GO:0007369] Sources: GOC:ascb_2009, GOC:dph, GOC:tb Definition: The change in form that occurs when an epithelial cell progresses from it initial formation to its mature state, contributing to the process of gastrulation.